{
  "term_id": "GO:0005833",
  "gene_symbol": "HBE1",
  "gene_name": "Hemoglobin subunit epsilon",
  "gene": "UniProtKB:P02100",
  "term_label": "hemoglobin complex"
}